maturation of SSU-rRNA from tricistronic rRNA transcript (SSU-rRNA, LSU-rRNA,5S) [GO:0002109] (biological process) Sources: GOC:curators Definition: Any process involved in the maturation of a precursor Small SubUnit (SSU) ribosomal RNA (rRNA) molecule into a mature SSU-rRNA molecule from the pre-rRNA molecule originally produced as a tricistronic rRNA transcript that contains the Small Subunit (SSU) rRNA, Large Subunit (LSU) the 5S rRNA in that order from 5' to 3' along the primary transcript. Relationships: is a type of maturation of SSU-rRNA [GO:0030490]